{
  "term_id": "GO:0051382",
  "gene": "UniProtKB:Q03188",
  "term_label": "kinetochore assembly",
  "gene_name": "Centromere protein C",
  "gene_symbol": "CENPC"
}